{
  "gene_symbol": "SEPTIN8",
  "gene_name": "Septin-8",
  "gene": "UniProtKB:Q92599",
  "term_id": "GO:0060090",
  "term_label": "molecular adaptor activity"
}